homoiothermy [GO:0042309] (biological process) Definition: Any homoeostatic process in which an organism maintains its internal body temperature at a relatively constant value. This is achieved by using metabolic processes to counteract fluctuations in the temperature of the environment. Relationships: is a type of GO:0001659 Also known as: antifreeze activity, ice nucleation activity, ice nucleation inhibitor activity Sources: ISBN:0192801023